{
  "gene_name": "Steroid transmembrane transporter SLC22A24",
  "gene_symbol": "SLC22A24",
  "gene": "UniProtKB:Q8N4F4",
  "term_id": "UNKNOWN:0003",
  "term_label": "Unknown cellular component"
}